{
  "term_id": "UNKNOWN:0002",
  "gene_symbol": "CCDC61",
  "term_label": "Unknown biological process",
  "gene_name": "Centrosomal protein CCDC61",
  "gene": "UniProtKB:Q9Y6R9"
}